lutropin-choriogonadotropic hormone receptor binding [GO:0031775] (molecular function) Relationships: is_a GO:0001664 Also known as: lutropin-choriogonadotropic hormone receptor ligand Definition: Binding to a lutropin-choriogonadotropic hormone receptor. Sources: GOC:mah, GOC:nln